{
  "gene": "UniProtKB:P20815",
  "term_id": "UNKNOWN:0003",
  "term_label": "Unknown cellular component",
  "gene_name": "Cytochrome P450 3A5",
  "gene_symbol": "CYP3A5"
}